negative regulation of neuron projection development [GO:0010977] (biological process) Definition: Any process that decreases the rate, frequency or extent of neuron projection development. Neuron projection development is the process whose specific outcome is the progression of a neuron projection over time, from its formation to the mature structure. A neuron projection is any process extending from a neural cell, such as axons or dendrites (collectively called neurites). Also known as: negative regulation of neurite biosynthesis, negative regulation of neurite development, negative regulation of neurite formation, negative regulation of neurite growth, growth cone collapse Relationships: is a type of regulation of neuron projection development [GO:0010975]; is a type of negative regulation of cell projection organization [GO:0031345]; negatively regulates neuron projection development [GO:0031175] Sources: GOC:dph, GOC:tb Subtypes: negative regulation of axonogenesis [GO:0050771], negative regulation of dendritic spine morphogenesis [GO:0061002], negative regulation of neuron projection regeneration [GO:0070571], negative regulation of axon guidance [GO:1902668], negative regulation of dendrite development [GO:2000171]